{
  "gene_name": "Transmembrane protein 138",
  "gene": "UniProtKB:Q9NPI0",
  "term_label": "cilium",
  "term_id": "GO:0005929",
  "gene_symbol": "TMEM138"
}